{
  "term_label": "Unknown cellular component",
  "gene_name": "MFS-type transporter SLC18B1",
  "term_id": "UNKNOWN:0003",
  "gene_symbol": "SLC18B1",
  "gene": "UniProtKB:Q6NT16"
}